{
  "gene_symbol": "ARSH",
  "gene": "UniProtKB:Q5FYA8",
  "gene_name": "Arylsulfatase H",
  "term_id": "UNKNOWN:0002",
  "term_label": "Unknown biological process"
}